{
  "term_label": "GTPase activity",
  "gene_name": "Ras-related protein Rab-37",
  "gene": "UniProtKB:Q96AX2",
  "term_id": "GO:0003924",
  "gene_symbol": "RAB37"
}